regulation of dipeptide transmembrane transport [GO:2001148] (BP) Subtypes: GO:2001149, GO:2001150 Sources: GOC:obol Also known as: regulation of dipeptide membrane transport Relationships: is a type of GO:0034762; is a type of regulation of dipeptide transport [GO:0090089]; regulates dipeptide transmembrane transport [GO:0035442] Definition: Any process that modulates the frequency, rate or extent of dipeptide transmembrane transport.